{
  "gene": "UniProtKB:Q9NPB0",
  "term_id": "GO:0005783",
  "gene_symbol": "SAYSD1",
  "gene_name": "SAYSvFN domain-containing protein 1",
  "term_label": "endoplasmic reticulum"
}